{
  "gene": "UniProtKB:Q8TED0",
  "term_label": "positive regulation of transcription by RNA polymerase I",
  "gene_symbol": "UTP15",
  "gene_name": "U3 small nucleolar RNA-associated protein 15 homolog",
  "term_id": "GO:0045943"
}